{
  "term_label": "ubiquitin binding",
  "gene_name": "Cyclin-dependent kinases regulatory subunit 1",
  "gene": "UniProtKB:P61024",
  "term_id": "GO:0043130",
  "gene_symbol": "CKS1B"
}